{
  "gene": "UniProtKB:Q3MIX3",
  "term_id": "UNKNOWN:0003",
  "term_label": "Unknown cellular component",
  "gene_name": "Uncharacterized aarF domain-containing protein kinase 5",
  "gene_symbol": "ADCK5"
}